{
  "term_id": "GO:0031763",
  "gene": "UniProtKB:P22466",
  "gene_name": "Galanin peptides",
  "term_label": "galanin receptor binding",
  "gene_symbol": "GAL"
}